{
  "term_label": "Unknown biological process",
  "gene_name": "Pseudouridine-5'-phosphatase",
  "term_id": "UNKNOWN:0002",
  "gene_symbol": "PUDP",
  "gene": "UniProtKB:Q08623"
}